negative regulation of post-transcriptional gene silencing [GO:0060149] (biological process) Definition: Any process that decreases the frequency, rate or extent of the inactivation of gene expression by a posttranscriptional mechanism. Sources: GOC:dph Subtypes: GO:1900369 Relationships: is a type of positive regulation of gene expression [GO:0010628]; is a type of GO:0048519; is a type of GO:0060147; negatively regulates post-transcriptional gene silencing [GO:0016441] Also known as: negative regulation of posttranscriptional gene silencing